{
  "gene_name": "Collagen alpha-1(XXVIII) chain",
  "term_id": "GO:0030199",
  "gene": "UniProtKB:Q2UY09",
  "gene_symbol": "COL28A1",
  "term_label": "collagen fibril organization"
}